{
  "gene": "UniProtKB:Q9NRH3",
  "gene_symbol": "TUBG2",
  "term_label": "microtubule nucleation",
  "term_id": "GO:0007020",
  "gene_name": "Tubulin gamma-2 chain"
}